{
  "term_id": "GO:0009982",
  "term_label": "pseudouridine synthase activity",
  "gene": "UniProtKB:Q9Y606",
  "gene_symbol": "PUS1",
  "gene_name": "Pseudouridylate synthase 1 homolog"
}